{
  "term_label": "plasma membrane",
  "term_id": "GO:0005886",
  "gene_symbol": "ADGRD2",
  "gene_name": "Adhesion G-protein coupled receptor D2",
  "gene": "UniProtKB:Q7Z7M1"
}